negative regulation of cell cycle checkpoint [GO:1901977] (biological process) Also known as: down regulation of cell cycle checkpoint, down-regulation of cell cycle checkpoint, downregulation of cell cycle checkpoint, inhibition of cell cycle checkpoint, negative regulation of G1/S checkpoint, negative regulation of G1/S transition checkpoint References: PMID:23028116 Sources: GOC:TermGenie, GOC:mtg_cell_cycle Definition: Any process that stops, prevents or reduces the frequency, rate or extent of cell cycle checkpoint. Note: Note that this term should not be used for direct manual annotation as it should always be possible to specify the type of checkpoint (i.e mitotic spindle or DNA damage etc). Subtypes: GO:0090233, negative regulation of DNA damage checkpoint [GO:2000002] Relationships: is a type of regulation of cell cycle checkpoint [GO:1901976]; is a type of positive regulation of cell cycle phase transition [GO:1901989]; is a type of GO:1902532; RO_0002212 cell cycle checkpoint signaling [GO:0000075]